{
  "term_id": "GO:0004674",
  "gene": "UniProtKB:P53350",
  "gene_name": "Serine_threonine-protein kinase PLK1",
  "term_label": "protein serine/threonine kinase activity",
  "gene_symbol": "PLK1"
}